positive regulation of dendritic cell chemotaxis [GO:2000510] (BP) Definition: Any process that activates or increases the frequency, rate or extent of dendritic cell chemotaxis. Relationships: is a type of positive regulation of leukocyte chemotaxis [GO:0002690]; is_a positive regulation of mononuclear cell migration [GO:0071677]; is a type of regulation of dendritic cell chemotaxis [GO:2000508]; positively regulates dendritic cell chemotaxis [GO:0002407] Sources: GOC:obol Subtypes: GO:2000529